{
  "term_id": "GO:0004784",
  "gene": "UniProtKB:P04179",
  "gene_name": "Superoxide dismutase [Mn], mitochondrial",
  "term_label": "superoxide dismutase activity",
  "gene_symbol": "SOD2"
}